{
  "gene": "UniProtKB:P26640",
  "term_label": "valine-tRNA ligase activity",
  "term_id": "GO:0004832",
  "gene_symbol": "VARS1",
  "gene_name": "Valine--tRNA ligase"
}